{
  "gene_name": "Polyunsaturated fatty acid 5-lipoxygenase",
  "term_id": "GO:0019372",
  "gene_symbol": "ALOX5",
  "gene": "UniProtKB:P09917",
  "term_label": "lipoxygenase pathway"
}